{
  "gene_name": "Zinc finger protein 282",
  "gene": "UniProtKB:Q9UDV7",
  "gene_symbol": "ZNF282",
  "term_id": "GO:0006355",
  "term_label": "regulation of DNA-templated transcription"
}